{
  "gene": "UniProtKB:Q5GFL6",
  "gene_symbol": "VWA2",
  "gene_name": "von Willebrand factor A domain-containing protein 2",
  "term_label": "basement membrane",
  "term_id": "GO:0005604"
}